{
  "term_label": "mitochondrion",
  "gene_symbol": "LYRM4",
  "gene": "UniProtKB:Q9HD34",
  "term_id": "GO:0005739",
  "gene_name": "LYR motif-containing protein 4"
}